{
  "gene_symbol": "SLC4A7",
  "term_id": "GO:0055085",
  "term_label": "transmembrane transport",
  "gene_name": "Sodium bicarbonate cotransporter 3",
  "gene": "UniProtKB:Q9Y6M7"
}